arabinose transmembrane transport [GO:0015751] (biological process) Subtypes: L-arabinose transmembrane transport [GO:0042882] Sources: GOC:jl Relationships: is a type of pentose transmembrane transport [GO:0015750] Also known as: arabinose transport Definition: The process in which arabinose, a pentose monosaccharide that occurs in both D and L configurations, is transported across a lipid bilayer, from one side of a membrane to the other.